ion binding [GO:0043167] (molecular function) Relationships: is a type of GO:0036094 Subtypes: anion binding [GO:0043168], cation binding [GO:0043169] Sources: GOC:jl Also known as: atom binding Definition: Binding to an ion, a charged atoms or groups of atoms.